{
  "term_label": "L-amino acid transmembrane transporter activity",
  "gene_symbol": "SLC38A10",
  "term_id": "GO:0015179",
  "gene_name": "Putative sodium-coupled neutral amino acid transporter 10",
  "gene": "UniProtKB:Q9HBR0"
}